{
  "term_label": "transforming growth factor beta receptor signaling pathway",
  "term_id": "GO:0007179",
  "gene_name": "Forkhead box protein H1",
  "gene_symbol": "FOXH1",
  "gene": "UniProtKB:O75593"
}